regulation of butyryl-CoA catabolic process to butyrate [GO:1900500] (biological process) Also known as: regulation of butyryl-CoA catabolism to butyrate Sources: GOC:TermGenie, GOC:mengo_curators Subtypes: GO:1900501, positive regulation of butyryl-CoA catabolic process to butyrate [GO:1900502] Relationships: is a type of regulation of nucleobase-containing compound metabolic process [GO:0019219]; is a type of GO:0034248; is_a GO:0042304; is a type of regulation of sulfur metabolic process [GO:0042762]; is a type of GO:0050994; is a type of regulation of phosphorus metabolic process [GO:0051174]; regulates butyryl-CoA catabolic process to butyrate [GO:0044581] Definition: Any process that modulates the frequency, rate or extent of butyryl-CoA catabolic process to butyrate.